{
  "term_id": "GO:0007399",
  "gene_name": "Paired box protein Pax-2",
  "term_label": "nervous system development",
  "gene_symbol": "PAX2",
  "gene": "UniProtKB:Q02962"
}